{
  "gene_name": "Synaptobrevin homolog YKT6",
  "gene_symbol": "YKT6",
  "term_id": "GO:0005484",
  "gene": "UniProtKB:O15498",
  "term_label": "SNAP receptor activity"
}